{
  "gene_symbol": "PRO2289",
  "term_id": "UNKNOWN:0003",
  "gene": "UniProtKB:Q9P1D8",
  "gene_name": "Putative uncharacterized protein PRO2289",
  "term_label": "Unknown cellular component"
}